{
  "gene_name": "V-type proton ATPase subunit B, brain isoform",
  "gene_symbol": "ATP6V1B2",
  "term_id": "GO:0007035",
  "gene": "UniProtKB:P21281",
  "term_label": "vacuolar acidification"
}